{
  "gene_name": "Protein Niban 1",
  "term_id": "UNKNOWN:0001",
  "gene_symbol": "NIBAN1",
  "term_label": "Unknown molecular function",
  "gene": "UniProtKB:Q9BZQ8"
}